{
  "gene_symbol": "MIR7-3HG",
  "gene_name": "Putative uncharacterized protein encoded by MIR7-3HG",
  "term_label": "Unknown biological process",
  "term_id": "UNKNOWN:0002",
  "gene": "UniProtKB:Q8N6C7"
}